{
  "gene_symbol": "SPAG11B",
  "gene_name": "Sperm-associated antigen 11B",
  "term_label": "Unknown cellular component",
  "gene": "UniProtKB:Q08648",
  "term_id": "UNKNOWN:0003"
}